{
  "gene": "UniProtKB:O95199",
  "term_label": "Unknown biological process",
  "term_id": "UNKNOWN:0002",
  "gene_symbol": "RCBTB2",
  "gene_name": "RCC1 and BTB domain-containing protein 2"
}